regulation of leaf development [GO:2000024] (BP) Definition: Any process that modulates the frequency, rate or extent of leaf development. Subtypes: negative regulation of leaf development [GO:1905622], GO:1905623, regulation of trichome morphogenesis [GO:2000039] Sources: GOC:obol Relationships: is a type of regulation of developmental process [GO:0050793]; regulates leaf development [GO:0048366]